{
  "gene": "UniProtKB:Q5MAI5",
  "gene_symbol": "CDKL4",
  "term_id": "UNKNOWN:0002",
  "gene_name": "Cyclin-dependent kinase-like 4",
  "term_label": "Unknown biological process"
}